{
  "gene_name": "Cartilage matrix protein",
  "gene_symbol": "MATN1",
  "term_id": "UNKNOWN:0002",
  "term_label": "Unknown biological process",
  "gene": "UniProtKB:P21941"
}